{
  "gene_name": "Small nuclear ribonucleoprotein-associated proteins B and B'",
  "gene_symbol": "SNRPB",
  "term_label": "U4 snRNP",
  "term_id": "GO:0005687",
  "gene": "UniProtKB:P14678"
}